transcription open complex formation at RNA polymerase II promoter [GO:0001113] (biological process) Relationships: is a type of DNA-templated transcription open complex formation [GO:0001112]; is part of transcription initiation at RNA polymerase II promoter [GO:0006367] Regulation: regulated by regulation of transcription open complex formation at RNA polymerase II promoter [GO:0001177] References: PMID:15020047, PMID:18280161 Sources: GOC:txnOH Also known as: RNA polymerase II promoter melting, transcriptional open complex formation at RNA polymerase II promoter Definition: Any process involved in the melting of the DNA hybrid of the core promoter region within the transcriptional closed complex of an RNA polymerase II preinitiation complex (PIC) to produce an open complex where the DNA duplex around the transcription initiation site is unwound to form the transcription bubble.